{
  "term_label": "Unknown cellular component",
  "gene_symbol": "TAL1",
  "term_id": "UNKNOWN:0003",
  "gene_name": "T-cell acute lymphocytic leukemia protein 1",
  "gene": "UniProtKB:P17542"
}